{
  "term_label": "GTPase activity",
  "gene_name": "Ras-related protein Rab-3C",
  "gene": "UniProtKB:Q96E17",
  "gene_symbol": "RAB3C",
  "term_id": "GO:0003924"
}